light-driven active monoatomic ion transmembrane transporter activity [GO:0015454] (molecular function) References: PMID:23994288, PMID:26442282 Sources: GOC:mtg_transport Also known as: light-driven active ion transmembrane transporter activity, light absorption-driven transporter, light-driven pumps, light-driven active transmembrane transporter activity Definition: Active transport of an ion across a membrane, driven by light. Relationships: is_a active monoatomic ion transmembrane transporter activity [GO:0022853]